{
  "term_label": "DNA damage response, signal transduction by p53 class mediator",
  "gene_symbol": "FOXM1",
  "gene_name": "Forkhead box protein M1",
  "term_id": "GO:0030330",
  "gene": "UniProtKB:Q08050"
}